{
  "term_label": "cytosol",
  "gene_symbol": "ASPA",
  "term_id": "GO:0005829",
  "gene_name": "Aspartoacylase",
  "gene": "UniProtKB:P45381"
}